{
  "term_label": "C-C chemokine receptor activity",
  "gene": "UniProtKB:P46094",
  "gene_symbol": "XCR1",
  "term_id": "GO:0016493",
  "gene_name": "Chemokine XC receptor 1"
}